{
  "term_id": "GO:0019626",
  "term_label": "short-chain fatty acid catabolic process",
  "gene_symbol": "CES1P1",
  "gene_name": "Putative inactive carboxylesterase 4",
  "gene": "UniProtKB:Q9UKY3"
}